{
  "term_id": "GO:1903940",
  "gene": "UniProtKB:Q8TB45",
  "gene_symbol": "DEPTOR",
  "gene_name": "DEP domain-containing mTOR-interacting protein",
  "term_label": "negative regulation of TORC2 signaling"
}